{
  "gene_name": "Protein YAE1 homolog",
  "term_id": "UNKNOWN:0001",
  "gene": "UniProtKB:Q9NRH1",
  "gene_symbol": "YAE1",
  "term_label": "Unknown molecular function"
}